{
  "term_label": "U4 snRNP",
  "gene_name": "U4_U6 small nuclear ribonucleoprotein Prp31",
  "gene_symbol": "PRPF31",
  "term_id": "GO:0005687",
  "gene": "UniProtKB:Q8WWY3"
}